{
  "gene_name": "A-kinase anchor protein 4",
  "term_label": "protein kinase A binding",
  "gene": "UniProtKB:Q5JQC9",
  "term_id": "GO:0051018",
  "gene_symbol": "AKAP4"
}